{
  "term_id": "GO:0034154",
  "gene_symbol": "UNC93B1",
  "gene_name": "Protein unc-93 homolog B1",
  "term_label": "toll-like receptor 7 signaling pathway",
  "gene": "UniProtKB:Q9H1C4"
}